{
  "gene_name": "1-phosphatidylinositol 4,5-bisphosphate phosphodiesterase delta-3",
  "gene_symbol": "PLCD3",
  "gene": "UniProtKB:Q8N3E9",
  "term_id": "GO:0005886",
  "term_label": "plasma membrane"
}